{
  "gene_symbol": "SLC6A15",
  "term_label": "proline:sodium symporter activity",
  "gene": "UniProtKB:Q9H2J7",
  "term_id": "GO:0005298",
  "gene_name": "Sodium-dependent neutral amino acid transporter B(0)AT2"
}